{
  "gene_symbol": "CD101",
  "gene_name": "Immunoglobulin superfamily member 2",
  "term_label": "Unknown biological process",
  "gene": "UniProtKB:Q93033",
  "term_id": "UNKNOWN:0002"
}